proline binding [GO:1901973] (molecular function) Definition: Binding to proline. References: PMID:7730362 Sources: GOC:TermGenie, GOC:pm Relationships: is a type of amino acid binding [GO:0016597]; is a type of carboxylic acid binding [GO:0031406]; is a type of heterocyclic compound binding [GO:1901363]